{
  "term_id": "GO:0005615",
  "term_label": "extracellular space",
  "gene_symbol": "PCSK1N",
  "gene_name": "ProSAAS",
  "gene": "UniProtKB:Q9UHG2"
}